negative regulation of interleukin-35 production [GO:0070755] (biological process) Relationships: is a type of GO:0001818; is a type of GO:0070754; negatively regulates interleukin-35 production [GO:0070753] Definition: Any process that stops, prevents, or reduces the frequency, rate, or extent of interleukin-35 production. Also known as: down regulation of interleukin-35 production, down-regulation of interleukin-35 production, downregulation of interleukin-35 production, negative regulation of IL-35 production, inhibition of interleukin-35 production, negative regulation of interleukin-35 biosynthetic process Sources: GOC:mah